synaptic transmission, serotonergic [GO:0099153] (biological process) Sources: GOC:dos, GOC:dph Relationships: is_a chemical synaptic transmission [GO:0007268] Also known as: serotonergic synaptic transmission Definition: The vesicular release of serotonin from a presynapse, across a chemical synapse, the subsequent activation of serotonin receptors at the postsynapse of a target cell (neuron, muscle, or secretory cell) and the effects of this activation on the postsynaptic membrane potential and ionic composition of the postsynaptic cytosol. This process encompasses both spontaneous and evoked release of neurotransmitter and all parts of synaptic vesicle exocytosis. Evoked transmission starts with the arrival of an action potential at the presynapse.